{
  "gene_name": "CUGBP Elav-like family member 2",
  "term_id": "GO:0005634",
  "gene_symbol": "CELF2",
  "term_label": "nucleus",
  "gene": "UniProtKB:O95319"
}